{
  "gene_name": "Peroxisomal coenzyme A diphosphatase NUDT7",
  "term_id": "GO:0005777",
  "gene": "UniProtKB:P0C024",
  "term_label": "peroxisome",
  "gene_symbol": "NUDT7"
}